{
  "gene_name": "Chronophin",
  "gene_symbol": "PDXP",
  "term_label": "cytoplasm",
  "gene": "UniProtKB:Q96GD0",
  "term_id": "GO:0005737"
}